{
  "gene_symbol": "DLGAP4",
  "gene_name": "Disks large-associated protein 4",
  "gene": "UniProtKB:Q9Y2H0",
  "term_id": "GO:0050804",
  "term_label": "modulation of chemical synaptic transmission"
}